rRNA transcription [GO:0009303] (biological process) Definition: The synthesis of ribosomal RNA (rRNA), any RNA that forms part of the ribosomal structure, from a DNA template. Relationships: is a type of GO:0006351; is a type of rRNA metabolic process [GO:0016072] Subtypes: nucleolar large rRNA transcription by RNA polymerase I [GO:0042790], 5S class rRNA transcription by RNA polymerase III [GO:0042791], GO:0042794 Sources: GOC:jl, ISBN:0198506732 Also known as: rRNA biosynthesis, rRNA biosynthetic process, rRNA synthesis